{
  "term_label": "poly(A)+ mRNA export from nucleus",
  "gene_name": "NTF2-related export protein 1",
  "gene_symbol": "NXT1",
  "term_id": "GO:0016973",
  "gene": "UniProtKB:Q9UKK6"
}